peptide hormone binding [GO:0017046] (MF) Definition: Binding to a peptide with hormonal activity in animals. Sources: GOC:jl, ISBN:0198506732 Subtypes: insulin binding [GO:0043559], corticotropin-releasing hormone binding [GO:0051424], gonadotropin-releasing hormone binding [GO:0051448], thyrotropin-releasing hormone binding [GO:0051449], adipokinetic hormone binding [GO:0097004], GO:0097644, glucagon family peptide binding [GO:0120022], somatostatin binding [GO:0120023] Relationships: is a type of amide binding [GO:0033218]; is a type of hormone binding [GO:0042562] Also known as: polypeptide hormone binding